{
  "gene_name": "Protein Jumonji",
  "gene": "UniProtKB:Q92833",
  "gene_symbol": "JARID2",
  "term_label": "nucleus",
  "term_id": "GO:0005634"
}